{
  "term_label": "Unknown molecular function",
  "gene_symbol": "CHCHD10",
  "gene_name": "Coiled-coil-helix-coiled-coil-helix domain-containing protein 10, mitochondrial",
  "gene": "UniProtKB:Q8WYQ3",
  "term_id": "UNKNOWN:0001"
}